pyridoxine binding [GO:0070282] (molecular function) Relationships: is_a GO:0070279 Sources: CHEBI:16709, GOC:mah Definition: Binding to pyridoxine, 4,5-bis(hydroxymethyl)-2-methylpyridin-3-ol, a form of vitamin B6.